{
  "gene_name": "DDB1- and CUL4-associated factor 4",
  "term_label": "Unknown molecular function",
  "gene": "UniProtKB:Q8WV16",
  "term_id": "UNKNOWN:0001",
  "gene_symbol": "DCAF4"
}